{
  "gene": "UniProtKB:B4DH59",
  "term_id": "UNKNOWN:0002",
  "gene_symbol": "NBPF26",
  "gene_name": "Neuroblastoma breakpoint family member 26",
  "term_label": "Unknown biological process"
}